methyl-branched fatty acid metabolic process [GO:0097089] (biological process) Also known as: methyl-branched fatty acid metabolism Definition: The chemical reactions and pathways involving methyl-branched fatty acids, aliphatic monocarboxylic acids with methyl branches on the main chain. References: PMID:19933331 Sources: GOC:rs Relationships: is a type of fatty acid metabolic process [GO:0006631] Subtypes: methyl-branched fatty acid biosynthetic process [GO:1902321], GO:1903512